{
  "term_label": "Unknown cellular component",
  "term_id": "UNKNOWN:0003",
  "gene_symbol": "SPDYE8",
  "gene": "UniProtKB:P0DUD1",
  "gene_name": "Putative speedy protein E8"
}